{
  "gene": "UniProtKB:P11717",
  "term_label": "trans-Golgi network",
  "term_id": "GO:0005802",
  "gene_name": "Cation-independent mannose-6-phosphate receptor",
  "gene_symbol": "IGF2R"
}